{
  "term_label": "intraciliary transport involved in cilium assembly",
  "term_id": "GO:0035735",
  "gene_symbol": "DYNC2LI1",
  "gene_name": "Cytoplasmic dynein 2 light intermediate chain 1",
  "gene": "UniProtKB:Q8TCX1"
}